{
  "gene_symbol": "ABCG2",
  "term_label": "ATPase-coupled transmembrane transporter activity",
  "gene": "UniProtKB:Q9UNQ0",
  "term_id": "GO:0042626",
  "gene_name": "Broad substrate specificity ATP-binding cassette transporter ABCG2"
}